{
  "term_id": "GO:0098609",
  "gene_name": "Integrin alpha-10",
  "term_label": "cell-cell adhesion",
  "gene_symbol": "ITGA10",
  "gene": "UniProtKB:O75578"
}